{
  "term_id": "GO:0016192",
  "gene": "UniProtKB:P59780",
  "gene_name": "AP-3 complex subunit sigma-2",
  "gene_symbol": "AP3S2",
  "term_label": "vesicle-mediated transport"
}